{
  "gene_symbol": "MARK2",
  "term_id": "GO:0000226",
  "gene": "UniProtKB:Q7KZI7",
  "term_label": "microtubule cytoskeleton organization",
  "gene_name": "Serine_threonine-protein kinase MARK2"
}